cell budding [GO:0007114] (BP) Regulation: RO_0002211 by regulation of cell budding [GO:0007116]; negatively regulated by negative regulation of cell budding [GO:0045781]; positively regulated by GO:0045782 Definition: A form of asexual reproduction, occurring in certain bacteria and fungi (e.g. yeasts) and some primitive animals in which an individual arises from a daughter cell formed by pinching off a part of the parent cell. The budlike outgrowths so formed may sometimes remain attached to the parent cell. Relationships: is_a asexual reproduction [GO:0019954]; is a type of reproductive process in single-celled organism [GO:0022413]; is a type of cell division [GO:0051301] Sources: ISBN:0198506732 Also known as: budding Subtypes: GO:0007120, bipolar cellular bud site selection [GO:0007121]